{
  "gene_name": "Cystatin-9-like",
  "gene_symbol": "CST9L",
  "term_label": "antimicrobial humoral response",
  "gene": "UniProtKB:Q9H4G1",
  "term_id": "GO:0019730"
}